{
  "term_label": "nucleoside triphosphate biosynthetic process",
  "gene_name": "Adenylate kinase 4, mitochondrial",
  "gene": "UniProtKB:P27144",
  "gene_symbol": "AK4",
  "term_id": "GO:0009142"
}